{
  "gene_name": "Ankyrin repeat and SOCS box protein 4",
  "term_label": "Unknown cellular component",
  "gene_symbol": "ASB4",
  "term_id": "UNKNOWN:0003",
  "gene": "UniProtKB:Q9Y574"
}